neutrophil clearance [GO:0097350] (biological process) References: PMID:21957127 Sources: GOC:BHF Definition: The selective elimination of senescent neutrophils from the body by autoregulatory mechanisms. Relationships: is a type of apoptotic cell clearance [GO:0043277]; is part of GO:0001780; has part GO:0006909